luteinization [GO:0001553] (biological process) Also known as: luteal phase Sources: https://www.ncbi.nlm.nih.gov/books/NBK279054/ Definition: The set of processes resulting in differentiation of theca and granulosa cells into luteal cells and in the formation of a corpus luteum after ovulation. Relationships: is a type of ovulation cycle process [GO:0022602]; is part of female gonad development [GO:0008585]